{
  "gene_name": "Emopamil-binding protein-like",
  "term_label": "Unknown molecular function",
  "term_id": "UNKNOWN:0001",
  "gene_symbol": "EBPL",
  "gene": "UniProtKB:Q9BY08"
}